{
  "term_label": "cytoplasm",
  "gene_name": "Glucose-dependent insulinotropic receptor",
  "term_id": "GO:0005737",
  "gene_symbol": "GPR119",
  "gene": "UniProtKB:Q8TDV5"
}